response to isooctane [GO:1902788] (biological process) Relationships: is a type of GO:1902778 Definition: Any process that results in a change in state or activity of a cell or an organism (in terms of movement, secretion, enzyme production, gene expression, etc.) as a result of an isooctane stimulus. Subtypes: cellular response to isooctane [GO:1902789] References: PMID:22328008 Sources: GOC:TermGenie, GOC:mengo_curators, GO_REF:0000071